positive regulation of tRNA metabolic process [GO:1903328] (biological process) Subtypes: positive regulation of tRNA catabolic process [GO:1902372], positive regulation of tRNA processing [GO:2000237] Sources: GOC:TermGenie, GOC:vw, GO_REF:0000058 Definition: Any process that activates or increases the frequency, rate or extent of tRNA metabolic process. Also known as: positive regulation of tRNA metabolism, up regulation of tRNA metabolic process, up regulation of tRNA metabolism, up-regulation of tRNA metabolic process, up-regulation of tRNA metabolism, upregulation of tRNA metabolic process, upregulation of tRNA metabolism, activation of tRNA metabolic process, activation of tRNA metabolism Relationships: is a type of positive regulation of RNA metabolic process [GO:0051254]; is a type of regulation of tRNA metabolic process [GO:1903326]; positively regulates GO:0006399